{
  "gene": "UniProtKB:Q8NDA2",
  "term_label": "plasma membrane",
  "gene_symbol": "HMCN2",
  "term_id": "GO:0005886",
  "gene_name": "Hemicentin-2"
}